{
  "term_label": "extracellular space",
  "gene_symbol": "LGI4",
  "gene_name": "Leucine-rich repeat LGI family member 4",
  "gene": "UniProtKB:Q8N135",
  "term_id": "GO:0005615"
}